{
  "gene_name": "Fanconi anemia group D2 protein",
  "term_label": "mitotic intra-S DNA damage checkpoint signaling",
  "gene_symbol": "FANCD2",
  "gene": "UniProtKB:Q9BXW9",
  "term_id": "GO:0031573"
}